regulation of superoxide metabolic process [GO:0090322] (biological process) Relationships: is a type of regulation of reactive oxygen species metabolic process [GO:2000377]; RO_0002211 superoxide metabolic process [GO:0006801] Subtypes: regulation of superoxide anion generation [GO:0032928], regulation of removal of superoxide radicals [GO:2000121] Also known as: regulation of superoxide metabolism Definition: Any process that modulates the rate, frequency, or extent of superoxide metabolism, the chemical reactions and pathways involving superoxide, the superoxide anion O2- (superoxide free radical), or any compound containing this species. Sources: GOC:tb